{
  "gene_name": "Trace amine-associated receptor 6",
  "gene_symbol": "TAAR6",
  "gene": "UniProtKB:Q96RI8",
  "term_label": "G protein-coupled receptor signaling pathway",
  "term_id": "GO:0007186"
}